{
  "gene_name": "Lactase_phlorizin hydrolase",
  "gene_symbol": "LCT",
  "gene": "UniProtKB:P09848",
  "term_id": "GO:0000016",
  "term_label": "lactase activity"
}